{
  "gene": "UniProtKB:Q86T65",
  "gene_symbol": "DAAM2",
  "gene_name": "Disheveled-associated activator of morphogenesis 2",
  "term_id": "UNKNOWN:0003",
  "term_label": "Unknown cellular component"
}